positive regulation of posterior neural plate formation by fibroblast growth factor receptor signaling pathway [GO:0060787] (biological process) Relationships: is a type of fibroblast growth factor receptor signaling pathway [GO:0008543]; is a type of regulation of embryonic development [GO:0045995]; is a type of positive regulation of morphogenesis of an epithelium [GO:1905332]; is a type of regulation of animal organ morphogenesis [GO:2000027]; positively regulates posterior neural plate formation [GO:0090018] Sources: GOC:dph, GOC:sdb_2009, GOC:tb Definition: Any process that increases the rate or extent of the formation of the posterior neural plate, the posterior end of the flat, thickened layer of ectodermal cells known as the neural plate. Also known as: positive regulation of posterior neural plate formation by fibroblast growth factor receptor signalling pathway, positive regulation of posterior neural plate formation by FGF receptor signaling pathway